{
  "gene_symbol": "STARD10",
  "term_id": "GO:0046581",
  "gene": "UniProtKB:Q9Y365",
  "gene_name": "START domain-containing protein 10",
  "term_label": "intercellular canaliculus"
}